{
  "gene_name": "Ras-GEF domain-containing family member 1B",
  "term_label": "guanyl-nucleotide exchange factor activity",
  "gene": "UniProtKB:Q0VAM2",
  "term_id": "GO:0005085",
  "gene_symbol": "RASGEF1B"
}